{
  "gene_symbol": "IL3RA",
  "term_label": "positive regulation of cell population proliferation",
  "gene": "UniProtKB:P26951",
  "term_id": "GO:0008284",
  "gene_name": "Interleukin-3 receptor subunit alpha"
}